{
  "term_id": "GO:0005634",
  "gene_name": "Peptidyl-prolyl cis-trans isomerase NIMA-interacting 4",
  "gene_symbol": "PIN4",
  "gene": "UniProtKB:Q9Y237",
  "term_label": "nucleus"
}